{
  "gene_symbol": "CLNK",
  "gene": "UniProtKB:Q7Z7G1",
  "term_label": "cytoplasm",
  "term_id": "GO:0005737",
  "gene_name": "Cytokine-dependent hematopoietic cell linker"
}